transforming growth factor beta receptor binding [GO:0005160] (molecular function) Subtypes: GO:0005114, type I transforming growth factor beta receptor binding [GO:0034713], type III transforming growth factor beta receptor binding [GO:0034714] Sources: GOC:ai Also known as: TGF-beta receptor binding, TGFbeta receptor binding, transforming growth factor beta, transforming growth factor beta receptor ligand, activin, inhibin, transforming growth factor beta ligand binding to type I receptor, transforming growth factor beta ligand binding to type II receptor, transforming growth factor beta receptor anchoring activity Definition: Binding to a transforming growth factor beta receptor. Relationships: is a type of GO:0005126